{
  "gene_symbol": "GRIN3B",
  "term_id": "GO:1904315",
  "gene_name": "Glutamate receptor ionotropic, NMDA 3B",
  "gene": "UniProtKB:O60391",
  "term_label": "transmitter-gated monoatomic ion channel activity involved in regulation of postsynaptic membrane potential"
}